{
  "gene_symbol": "PRAMEF15",
  "gene": "UniProtKB:P0DUQ1",
  "term_label": "proteasome-mediated ubiquitin-dependent protein catabolic process",
  "gene_name": "PRAME family member 15",
  "term_id": "GO:0043161"
}